{
  "gene_name": "Dynamin-like 120 kDa protein, mitochondrial",
  "term_label": "GTPase activity",
  "term_id": "GO:0003924",
  "gene_symbol": "OPA1",
  "gene": "UniProtKB:O60313"
}